{
  "term_id": "GO:0003735",
  "gene": "UniProtKB:Q07020",
  "term_label": "structural constituent of ribosome",
  "gene_symbol": "RPL18",
  "gene_name": "Large ribosomal subunit protein eL18"
}